{
  "term_label": "phagocytic cup",
  "gene_name": "Rab11 family-interacting protein 2",
  "gene": "UniProtKB:Q7L804",
  "gene_symbol": "RAB11FIP2",
  "term_id": "GO:0001891"
}